{
  "term_label": "Unknown cellular component",
  "gene_symbol": "NAT16",
  "gene": "UniProtKB:Q8N8M0",
  "term_id": "UNKNOWN:0003",
  "gene_name": "Probable N-acetyltransferase 16"
}